{
  "term_label": "endocytosis",
  "gene": "UniProtKB:Q9H4E5",
  "gene_name": "Rho-related GTP-binding protein RhoJ",
  "gene_symbol": "RHOJ",
  "term_id": "GO:0006897"
}